{
  "gene": "UniProtKB:Q5T035",
  "term_id": "UNKNOWN:0003",
  "gene_name": "Putative uncharacterized protein FAM120A2P",
  "gene_symbol": "FAM120A2P",
  "term_label": "Unknown cellular component"
}